{
  "term_id": "GO:0043484",
  "term_label": "regulation of RNA splicing",
  "gene_symbol": "ESRP2",
  "gene_name": "Epithelial splicing regulatory protein 2",
  "gene": "UniProtKB:Q9H6T0"
}